{
  "gene": "UniProtKB:Q96J02",
  "gene_name": "E3 ubiquitin-protein ligase Itchy homolog",
  "gene_symbol": "ITCH",
  "term_id": "GO:0005737",
  "term_label": "cytoplasm"
}